{
  "gene_name": "Retinoic acid receptor alpha",
  "gene_symbol": "RARA",
  "gene": "UniProtKB:P10276",
  "term_label": "positive regulation of transcription by RNA polymerase II",
  "term_id": "GO:0045944"
}